{
  "gene": "UniProtKB:Q86UE6",
  "gene_name": "Leucine-rich repeat transmembrane neuronal protein 1",
  "term_id": "GO:0051965",
  "term_label": "positive regulation of synapse assembly",
  "gene_symbol": "LRRTM1"
}